{
  "gene_symbol": "NUAK1",
  "term_label": "Unknown biological process",
  "term_id": "UNKNOWN:0002",
  "gene_name": "NUAK family SNF1-like kinase 1",
  "gene": "UniProtKB:O60285"
}